{
  "term_id": "GO:0005768",
  "term_label": "endosome",
  "gene": "UniProtKB:Q96B67",
  "gene_name": "Arrestin domain-containing protein 3",
  "gene_symbol": "ARRDC3"
}